{
  "gene_name": "Tripeptidyl-peptidase 1",
  "term_label": "central nervous system development",
  "term_id": "GO:0007417",
  "gene_symbol": "TPP1",
  "gene": "UniProtKB:O14773"
}